{
  "term_label": "dipeptidyl-peptidase activity",
  "gene": "UniProtKB:Q9NY33",
  "gene_name": "Dipeptidyl peptidase 3",
  "gene_symbol": "DPP3",
  "term_id": "GO:0008239"
}